phosphatidylinositol catabolic process [GO:0031161] (biological process) Definition: The chemical reactions and pathways resulting in the breakdown of phosphatidylinositol, any glycophospholipid with its sn-glycerol 3-phosphate residue is esterified to the 1-hydroxyl group of 1D-myo-inositol. Also known as: PtdIns catabolic process, PtdIns catabolism, phosphatidylinositol breakdown, phosphatidylinositol catabolism, phosphatidylinositol degradation Subtypes: GO:1902634, 1-phosphatidyl-1D-myo-inositol 3,5-bisphosphate catabolic process [GO:1903101] Relationships: is a type of GO:0046475; is_a phosphatidylinositol metabolic process [GO:0046488] Sources: GOC:mah